{
  "gene_name": "Mas-related G-protein coupled receptor member X3",
  "gene_symbol": "MRGPRX3",
  "gene": "UniProtKB:Q96LB0",
  "term_label": "plasma membrane",
  "term_id": "GO:0005886"
}